{
  "gene_name": "Uncharacterized protein C15orf39",
  "term_id": "UNKNOWN:0001",
  "gene": "UniProtKB:Q6ZRI6",
  "term_label": "Unknown molecular function",
  "gene_symbol": "C15orf39"
}